{
  "term_id": "GO:0007156",
  "gene_symbol": "SDK1",
  "term_label": "homophilic cell-cell adhesion",
  "gene": "UniProtKB:Q7Z5N4",
  "gene_name": "Protein sidekick-1"
}